{
  "term_label": "cilium movement involved in cell motility",
  "term_id": "GO:0060294",
  "gene_name": "Cytoplasmic dynein 2 heavy chain 1",
  "gene_symbol": "DYNC2H1",
  "gene": "UniProtKB:Q8NCM8"
}